{
  "term_label": "Unknown cellular component",
  "gene_symbol": "FAM90A27P",
  "term_id": "UNKNOWN:0003",
  "gene": "UniProtKB:A6NNH2",
  "gene_name": "Protein FAM90A27P"
}